{
  "term_id": "UNKNOWN:0003",
  "term_label": "Unknown cellular component",
  "gene": "UniProtKB:Q96KR7",
  "gene_symbol": "PHACTR3",
  "gene_name": "Phosphatase and actin regulator 3"
}